{
  "term_label": "cell adhesion",
  "gene_symbol": "ICAM3",
  "gene": "UniProtKB:P32942",
  "gene_name": "Intercellular adhesion molecule 3",
  "term_id": "GO:0007155"
}